kappa-carrageenase activity [GO:0033918] (molecular function) Definition: Catalysis of the endohydrolysis of 1,4-beta-D-linkages between D-galactose 4-sulfate and 3,6-anhydro-D-galactose in kappa-carrageenans. Also known as: kappa-carrageenan 4-beta-D-glycanohydrolase (configuration-retaining) activity, kappa-carrageenan 4-beta-D-glycanohydrolase activity Relationships: is a type of hydrolase activity, hydrolyzing O-glycosyl compounds [GO:0004553] Sources: EC:3.2.1.83